{
  "term_id": "UNKNOWN:0002",
  "term_label": "Unknown biological process",
  "gene_name": "Cell surface hyaluronidase",
  "gene": "UniProtKB:Q9UHN6",
  "gene_symbol": "CEMIP2"
}